4-chlorobenzoate-CoA ligase activity [GO:0018861] (molecular function) Relationships: is a type of CoA-ligase activity [GO:0016405]; is a type of acid-thiol ligase activity [GO:0016878] Also known as: 4-chlorobenzoate:CoA ligase activity Sources: EC:6.2.1.33 Definition: Catalysis of the reaction: 4-chlorobenzoate + CoA + ATP = 4-chlorobenzoyl-CoA + AMP + diphosphate. This reaction requires magnesium and is part of the bacterial 2,4-dichlorobenzoate degradation pathway.